{
  "gene_symbol": "HERV-K104",
  "term_label": "Unknown biological process",
  "gene": "UniProtKB:P63124",
  "gene_name": "Endogenous retrovirus group K member 104 Pro protein",
  "term_id": "UNKNOWN:0002"
}